peptide biosynthetic process [GO:0043043] (BP) Subtypes: antimicrobial peptide biosynthetic process [GO:0002777], GO:0002936, nonribosomal peptide biosynthetic process [GO:0019184], peptide antibiotic biosynthetic process [GO:0030651] Relationships: is a type of peptide metabolic process [GO:0006518]; is a type of GO:0009058 Sources: GOC:dph, GOC:jl Definition: The chemical reactions and pathways resulting in the formation of peptides, compounds of 2 or more (but usually less than 100) amino acids where the alpha carboxyl group of one is bound to the alpha amino group of another. This may include the translation of a precursor protein and its subsequent processing into a functional peptide. Also known as: peptide anabolism, peptide biosynthesis, peptide formation, peptide synthesis